{
  "gene_name": "DCN1-like protein 2",
  "gene_symbol": "DCUN1D2",
  "term_id": "GO:0032182",
  "gene": "UniProtKB:Q6PH85",
  "term_label": "ubiquitin-like protein binding"
}